{
  "term_label": "nucleus",
  "gene": "UniProtKB:Q96FX7",
  "gene_name": "tRNA (adenine(58)-N(1))-methyltransferase catalytic subunit TRMT61A",
  "term_id": "GO:0005634",
  "gene_symbol": "TRMT61A"
}